{
  "term_id": "GO:0005737",
  "gene_name": "Exportin-T",
  "gene": "UniProtKB:O43592",
  "term_label": "cytoplasm",
  "gene_symbol": "XPOT"
}